positive regulation of biological process [GO:0048518] (biological process) Relationships: is a type of regulation of biological process [GO:0050789]; positively regulates biological_process [GO:0008150] Definition: Any process that activates or increases the frequency, rate or extent of a biological process. Biological processes are regulated by many means; examples include the control of gene expression, protein modification or interaction with a protein or substrate molecule. Also known as: positive regulation of physiological process, up regulation of biological process, up-regulation of biological process, upregulation of biological process, activation of biological process, stimulation of biological process Subtypes: positive regulation of immune system process [GO:0002684], positive regulation of signaling [GO:0023056], positive regulation of border follicle cell delamination [GO:0030711], positive regulation of cellular pH reduction [GO:0032849], positive regulation of locomotion [GO:0040017], positive regulation of circadian rhythm [GO:0042753], positive regulation of formation of structure involved in a symbiotic process [GO:0044149], GO:0045760, positive regulation of growth [GO:0045927], GO:0048087, positive regulation of cellular process [GO:0048522], GO:0048524, GO:0048584, positive regulation of transport [GO:0051050], positive regulation of developmental process [GO:0051094], GO:0051240, positive regulation of fibrinolysis [GO:0051919], positive regulation of post-transcriptional gene silencing [GO:0060148], positive regulation by symbiont of entry into host [GO:0075294], GO:0106428, positive regulation of transepithelial migration of symbiont in host [GO:0140471], positive regulation of hemostasis [GO:1900048], positive regulation of long-term synaptic depression [GO:1900454], positive regulation of membrane hyperpolarization [GO:1902632], GO:1902685, positive regulation of cardiac conduction [GO:1903781], positive regulation of protein localization [GO:1903829], positive regulation of membrane depolarization [GO:1904181], positive regulation of transformation of host cell by virus [GO:1904189], positive regulation of intracellular mRNA localization [GO:1904582], positive regulation of telomerase RNA localization to Cajal body [GO:1904874], GO:1904912, positive regulation of establishment of protein-containing complex localization to telomere [GO:1904915], GO:1904951, positive regulation of membrane repolarization during cardiac muscle cell action potential [GO:1905033], positive regulation of short-term synaptic potentiation [GO:1905514], positive regulation of lipid localization [GO:1905954], positive regulation of reproductive process [GO:2000243] Sources: GOC:jid